{
  "gene": "UniProtKB:Q96K31",
  "gene_symbol": "C8orf76",
  "term_id": "UNKNOWN:0001",
  "term_label": "Unknown molecular function",
  "gene_name": "Uncharacterized protein C8orf76"
}